{
  "term_id": "GO:1903078",
  "gene_name": "Calcium and integrin-binding protein 1",
  "term_label": "positive regulation of protein localization to plasma membrane",
  "gene": "UniProtKB:Q99828",
  "gene_symbol": "CIB1"
}